{
  "gene_name": "Olfactory receptor 5M11",
  "gene_symbol": "OR5M11",
  "gene": "UniProtKB:Q96RB7",
  "term_label": "Unknown biological process",
  "term_id": "UNKNOWN:0002"
}